{
  "term_label": "Unknown molecular function",
  "gene_symbol": "Q6ZRU5",
  "gene_name": "Putative uncharacterized protein FLJ46089",
  "gene": "UniProtKB:Q6ZRU5",
  "term_id": "UNKNOWN:0001"
}